{
  "term_id": "GO:0003712",
  "gene": "UniProtKB:Q9HAZ2",
  "gene_symbol": "PRDM16",
  "gene_name": "Histone-lysine N-methyltransferase PRDM16",
  "term_label": "transcription coregulator activity"
}